{
  "gene_symbol": "DDX59",
  "term_id": "UNKNOWN:0003",
  "gene": "UniProtKB:Q5T1V6",
  "gene_name": "Probable ATP-dependent RNA helicase DDX59",
  "term_label": "Unknown cellular component"
}